peptidase activity [GO:0008233] (molecular function) Subtypes: endopeptidase activity [GO:0004175], GO:0004176, GO:0008234, serine-type peptidase activity [GO:0008236], metallopeptidase activity [GO:0008237], exopeptidase activity [GO:0008238], GO:0008242, ubiquitin-like protein peptidase activity [GO:0019783], aspartic-type peptidase activity [GO:0070001], glutamic-type peptidase activity [GO:0070002], GO:0070003 Sources: EC:3.4.-.-, GOC:jl Definition: Catalysis of the hydrolysis of a peptide bond. A peptide bond is a covalent bond formed when the carbon atom from the carboxyl group of one amino acid shares electrons with the nitrogen atom from the amino group of a second amino acid. Also known as: hydrolase, acting on peptide bonds, peptide hydrolase activity, protease activity, peptidase activity, acting on D-amino acid peptides, peptidase activity, acting on L-amino acid peptides, proteinase activity Regulation: negatively regulated by negative regulation of peptidase activity [GO:0010466]; positively regulated by positive regulation of peptidase activity [GO:0010952]; positively regulated by peptidase activator activity [GO:0016504]; negatively regulated by peptidase inhibitor activity [GO:0030414]; regulated by regulation of peptidase activity [GO:0052547]; regulated by peptidase regulator activity [GO:0061134] Relationships: is a type of hydrolase activity [GO:0016787]; is a type of catalytic activity, acting on a protein [GO:0140096]